{
  "gene_name": "Small conductance calcium-activated potassium channel protein 1",
  "gene_symbol": "KCNN1",
  "gene": "UniProtKB:Q92952",
  "term_label": "calmodulin binding",
  "term_id": "GO:0005516"
}